{
  "gene_name": "Nurim",
  "gene": "UniProtKB:Q8IXM6",
  "gene_symbol": "NRM",
  "term_id": "UNKNOWN:0002",
  "term_label": "Unknown biological process"
}